{
  "term_id": "UNKNOWN:0003",
  "gene_symbol": "ANKRD49",
  "gene_name": "Ankyrin repeat domain-containing protein 49",
  "term_label": "Unknown cellular component",
  "gene": "UniProtKB:Q8WVL7"
}